endonucleolytic cleavage of tricistronic rRNA transcript (SSU-rRNA, 5.8S rRNA, LSU-rRNA) [GO:0000479] (biological process) References: PMID:10690410 Sources: GOC:curators Relationships: is a type of rRNA processing [GO:0006364] Subtypes: endonucleolytic cleavage in ITS1 to separate SSU-rRNA from 5.8S rRNA and LSU-rRNA from tricistronic rRNA transcript (SSU-rRNA, 5.8S rRNA, LSU-rRNA) [GO:0000447], cleavage in ITS2 between 5.8S rRNA and LSU-rRNA of tricistronic rRNA transcript (SSU-rRNA, 5.8S rRNA, LSU-rRNA) [GO:0000448], endonucleolytic cleavage to generate mature 3'-end of SSU-rRNA from (SSU-rRNA, 5.8S rRNA, LSU-rRNA) [GO:0000461], endonucleolytic cleavage in ITS1 upstream of 5.8S rRNA from tricistronic rRNA transcript (SSU-rRNA, 5.8S rRNA, LSU-rRNA) [GO:0000464], endonucleolytic cleavage in 3'-ETS of tricistronic rRNA transcript (SSU-rRNA, 5.8S rRNA, LSU-rRNA) [GO:0000471], endonucleolytic cleavage to generate mature 5'-end of SSU-rRNA from (SSU-rRNA, 5.8S rRNA, LSU-rRNA) [GO:0000472], GO:0000480 Definition: Endonucleolytic cleavage of a pre-rRNA molecule originally produced as a tricistronic rRNA transcript that contains the Small SubUnit (SSU) rRNA, the 5.8S rRNA, and the Large SubUnit (LSU) rRNA, in that order, from 5' to 3' along the primary transcript. Primary ribosomal RNA transcripts with three genes, in this order, are produced in the nuclei of many eukaryotic species, including S. cerevisiae.